{
  "gene_name": "Metalloreductase STEAP3",
  "gene_symbol": "STEAP3",
  "gene": "UniProtKB:Q658P3",
  "term_id": "GO:0005886",
  "term_label": "plasma membrane"
}